{
  "term_label": "positive regulation of programmed cell death",
  "gene_name": "Oxidoreductase HTATIP2",
  "term_id": "GO:0043068",
  "gene": "UniProtKB:Q9BUP3",
  "gene_symbol": "HTATIP2"
}